regulation of nematode male tail tip morphogenesis [GO:0110037] (biological process) Relationships: is_a regulation of anatomical structure morphogenesis [GO:0022603]; regulates GO:0045138 References: PMID:28068334 Sources: GOC:rz Definition: Any process that modulates the frequency, rate or extent of nematode male tail tip morphogenesis, the process in which the anatomical structure of the adult male tail tip is generated and organized. Subtypes: negative regulation of nematode male tail tip morphogenesis [GO:0110038], positive regulation of nematode male tail tip morphogenesis [GO:0110039]